{
  "term_label": "GTPase activator activity",
  "gene_name": "TBC1 domain family member 3E",
  "gene_symbol": "TBC1D3E",
  "term_id": "GO:0005096",
  "gene": "UniProtKB:A0A087X179"
}